{
  "gene_symbol": "SLC28A2",
  "term_id": "GO:0001895",
  "gene": "UniProtKB:O43868",
  "term_label": "retina homeostasis",
  "gene_name": "Sodium_nucleoside cotransporter 2"
}